{
  "term_id": "GO:0001228",
  "gene_symbol": "SOX14",
  "gene": "UniProtKB:O95416",
  "gene_name": "Transcription factor SOX-14",
  "term_label": "DNA-binding transcription activator activity, RNA polymerase II-specific"
}